{
  "gene": "UniProtKB:Q8NF86",
  "term_id": "GO:0004252",
  "term_label": "serine-type endopeptidase activity",
  "gene_symbol": "PRSS33",
  "gene_name": "Serine protease 33"
}